{
  "term_label": "regulation of transcription by RNA polymerase II",
  "gene_name": "Histone acetyltransferase KAT6B",
  "gene_symbol": "KAT6B",
  "term_id": "GO:0006357",
  "gene": "UniProtKB:Q8WYB5"
}